{
  "term_label": "RNA binding",
  "term_id": "GO:0003723",
  "gene_symbol": "RPL3L",
  "gene": "UniProtKB:Q92901",
  "gene_name": "Ribosomal protein uL3-like"
}